regulation of tendon cell differentiation [GO:2001049] (biological process) Sources: GOC:obol Definition: Any process that modulates the frequency, rate or extent of tendon cell differentiation. Relationships: is_a regulation of cell differentiation [GO:0045595]; regulates tendon cell differentiation [GO:0035990] Subtypes: negative regulation of tendon cell differentiation [GO:2001050], positive regulation of tendon cell differentiation [GO:2001051] Also known as: regulation of muscle attachment cell differentiation, regulation of tenocyte differentiation